{
  "term_label": "positive regulation of Wnt signaling pathway",
  "gene": "UniProtKB:Q96SW2",
  "term_id": "GO:0030177",
  "gene_symbol": "CRBN",
  "gene_name": "Protein cereblon"
}